{
  "gene_symbol": "DES",
  "gene_name": "Desmin",
  "gene": "UniProtKB:P17661",
  "term_id": "GO:0045109",
  "term_label": "intermediate filament organization"
}